{
  "gene_name": "Putative zinc finger protein 705G",
  "term_id": "GO:0005634",
  "gene": "UniProtKB:A8MUZ8",
  "term_label": "nucleus",
  "gene_symbol": "ZNF705G"
}